{
  "gene_symbol": "HS6ST3",
  "term_id": "UNKNOWN:0003",
  "gene": "UniProtKB:Q8IZP7",
  "term_label": "Unknown cellular component",
  "gene_name": "Heparan-sulfate 6-O-sulfotransferase 3"
}